{
  "gene_name": "Nuclear receptor-interacting protein 1",
  "gene": "UniProtKB:P48552",
  "term_id": "GO:0071392",
  "gene_symbol": "NRIP1",
  "term_label": "cellular response to estradiol stimulus"
}